{
  "gene_name": "Uncharacterized protein KRT10-AS1",
  "term_id": "UNKNOWN:0003",
  "term_label": "Unknown cellular component",
  "gene_symbol": "KRT10-AS1",
  "gene": "UniProtKB:Q8N816"
}